{
  "gene": "UniProtKB:O00755",
  "gene_name": "Protein Wnt-7a",
  "term_label": "neuron differentiation",
  "term_id": "GO:0030182",
  "gene_symbol": "WNT7A"
}